positive regulation of N-terminal peptidyl-lysine acetylation [GO:2000761] (biological process) Relationships: is a type of GO:1903319; is a type of positive regulation of peptidyl-lysine acetylation [GO:2000758]; is a type of GO:2000759; positively regulates N-terminal peptidyl-lysine acetylation [GO:0018076] Sources: GOC:obol Definition: Any process that activates or increases the frequency, rate or extent of N-terminal peptidyl-lysine acetylation.